{
  "gene_symbol": "ANKIB1",
  "term_id": "GO:0031624",
  "gene": "UniProtKB:Q9P2G1",
  "gene_name": "Ankyrin repeat and IBR domain-containing protein 1",
  "term_label": "ubiquitin conjugating enzyme binding"
}